negative regulation of memory T cell differentiation [GO:0043381] (biological process) Definition: Any process that stops, prevents, or reduces the rate of memory T cell differentiation. Relationships: is a type of negative regulation of immune effector process [GO:0002698]; is a type of regulation of memory T cell differentiation [GO:0043380]; is a type of GO:0045581; is a type of negative regulation of immune response [GO:0050777]; negatively regulates GO:0043379 Also known as: down regulation of memory T cell differentiation, down-regulation of memory T cell differentiation, downregulation of memory T cell differentiation, negative regulation of memory T lymphocyte differentiation, negative regulation of memory T-cell differentiation, negative regulation of memory T-lymphocyte differentiation, inhibition of memory T cell differentiation, negative regulation of memory T cell development Sources: ISBN:0781735149 Note: Note that immunologists typically use the word 'development' to refer to cells of B or T cell lineages undergoing the process that GO describes as 'cell differentiation'.